compound eye photoreceptor cell differentiation [GO:0001751] (biological process) Relationships: is a type of eye photoreceptor cell differentiation [GO:0001754]; is part of compound eye morphogenesis [GO:0001745] Definition: The process in which a relatively unspecialized cell acquires the specialized features of an eye photoreceptor cell. Regulation: regulated by regulation of compound eye photoreceptor cell differentiation [GO:0110116]; positively regulated by positive regulation of compound eye photoreceptor cell differentiation [GO:0110117]; negatively regulated by negative regulation of compound eye photoreceptor cell differentiation [GO:0110118] Sources: GOC:go_curators Subtypes: R8 cell differentiation [GO:0045465], R7 cell differentiation [GO:0045466], R1/R6 cell differentiation [GO:0048052], R2/R5 cell differentiation [GO:0048054], R3/R4 cell differentiation [GO:0048056]